negative regulation of dopamine biosynthetic process [GO:1903180] (biological process) Definition: Any process that stops, prevents or reduces the frequency, rate or extent of dopamine biosynthetic process. Also known as: down regulation of dopamine anabolism, down regulation of dopamine biosynthesis, down regulation of dopamine biosynthetic process, down regulation of dopamine formation, down regulation of dopamine synthesis, down-regulation of dopamine anabolism, down-regulation of dopamine biosynthesis, down-regulation of dopamine biosynthetic process, down-regulation of dopamine formation, down-regulation of dopamine synthesis, downregulation of dopamine anabolism, downregulation of dopamine biosynthesis, downregulation of dopamine biosynthetic process, downregulation of dopamine formation, downregulation of dopamine synthesis, negative regulation of dopamine anabolism, negative regulation of dopamine biosynthesis, negative regulation of dopamine formation, negative regulation of dopamine synthesis, inhibition of dopamine anabolism, inhibition of dopamine biosynthesis, inhibition of dopamine biosynthetic process, inhibition of dopamine formation, inhibition of dopamine synthesis Relationships: is a type of GO:0009890; is a type of negative regulation of dopamine metabolic process [GO:0045963]; is a type of regulation of dopamine biosynthetic process [GO:1903179]; negatively regulates dopamine biosynthetic process [GO:0042416] Sources: GOC:PARL, GOC:TermGenie, GOC:bf, GO_REF:0000058